{
  "term_id": "GO:0005634",
  "gene_name": "PR domain zinc finger protein 2",
  "gene": "UniProtKB:Q13029",
  "term_label": "nucleus",
  "gene_symbol": "PRDM2"
}